negative regulation of cellular senescence [GO:2000773] (biological process) Definition: Any process that stops, prevents or reduces the frequency, rate or extent of cellular senescence. Sources: GOC:BHF Relationships: is a type of negative regulation of cellular process [GO:0048523]; is a type of regulation of cellular senescence [GO:2000772]; negatively regulates GO:0090398